positive regulation of flavonol biosynthetic process [GO:1900386] (biological process) Definition: Any process that activates or increases the frequency, rate or extent of flavonol biosynthetic process. Relationships: is a type of GO:0009963; is a type of regulation of flavonol biosynthetic process [GO:1900384]; positively regulates flavonol biosynthetic process [GO:0051555] Also known as: up regulation of flavonol biosynthetic process, up-regulation of flavonol biosynthetic process, upregulation of flavonol biosynthetic process, activation of flavonol biosynthetic process Sources: GOC:TermGenie